{
  "term_label": "cytoplasm",
  "gene_name": "ADP-ribosylation factor 5",
  "gene_symbol": "ARF5",
  "term_id": "GO:0005737",
  "gene": "UniProtKB:P84085"
}